{
  "gene_symbol": "RDH13",
  "term_id": "GO:0005743",
  "gene": "UniProtKB:Q8NBN7",
  "term_label": "mitochondrial inner membrane",
  "gene_name": "Retinol dehydrogenase 13"
}